{
  "term_id": "GO:0050911",
  "gene_symbol": "OR2T1",
  "term_label": "detection of chemical stimulus involved in sensory perception of smell",
  "gene_name": "Olfactory receptor 2T1",
  "gene": "UniProtKB:O43869"
}